{
  "term_id": "GO:0003899",
  "gene_name": "DNA-directed RNA polymerase I subunit RPA12",
  "gene_symbol": "POLR1H",
  "term_label": "DNA-directed RNA polymerase activity",
  "gene": "UniProtKB:Q9P1U0"
}